positive regulation of forebrain neuron differentiation [GO:2000979] (biological process) Definition: Any process that activates or increases the frequency, rate or extent of forebrain neuron differentiation. Relationships: is a type of GO:0045666; is a type of regulation of forebrain neuron differentiation [GO:2000977]; positively regulates forebrain neuron differentiation [GO:0021879] Sources: GOC:obol